{
  "term_label": "trans-Golgi network membrane",
  "gene_symbol": "BAIAP3",
  "gene": "UniProtKB:O94812",
  "term_id": "GO:0032588",
  "gene_name": "BAI1-associated protein 3"
}